CRLF-CLCF1 complex [GO:0097058] (cellular component) Also known as: CLF-CLC complex References: PMID:10966616 Sources: GOC:BHF Relationships: is a type of GO:0032991; is part of extracellular region [GO:0005576] Definition: A heterodimeric protein complex that is composed of cardiotrophin-like cytokine factor 1 (product of the CLCF1 gene) and cytokine receptor-like factor 1 (product of the CRLF gene) and is secreted into the extracellular space. The CRLF-CLCF1 complex is a ligand for the ciliary neurotrophic factor (CNTF) receptor complex.